15-hydroxyprostaglandin dehydrogenase (NAD+) activity [GO:0016404] (molecular function) Sources: EC:1.1.1.141 Also known as: (5Z,13E)-(15S)-11alpha,15-dihydroxy-9-oxoprost-13-enoate:NAD+ 15-oxidoreductase activity, 11alpha,15-dihydroxy-9-oxoprost-13-enoate:NAD+ 15-oxidoreductase activity, 15-OH-PGDH, 15-hydroxyprostaglandin dehydrogenase activity, 15-hydroxyprostanoic dehydrogenase activity, NAD+-dependent 15-hydroxyprostaglandin dehydrogenase (type I), NAD-specific 15-hydroxyprostaglandin dehydrogenase activity, prostaglandin dehydrogenase activity Definition: Catalysis of the reaction: (5Z,13E)-(15S)-11-alpha,15-dihydroxy-9-oxoprost-13-enoate + NAD+ = (5Z,13E)-11-alpha-hydroxy-9,15-dioxoprost-13-enoate + NADH + H+. Relationships: is a type of oxidoreductase activity, acting on the CH-OH group of donors, NAD or NADP as acceptor [GO:0016616]